cellotriose transport [GO:2001096] (BP) Sources: GOC:mengo_curators Regulation: regulated by regulation of cellotriose transport [GO:1900285]; negatively regulated by negative regulation of cellotriose transport [GO:1900286]; positively regulated by GO:1900287 Definition: The directed movement of a cellotrioseacetate into, out of or within a cell, or between cells, by means of some agent such as a transporter or pore. Relationships: is a type of trisaccharide transport [GO:2001088]